regulation of isopentenyl diphosphate biosynthetic process, mevalonate pathway [GO:2001210] (biological process) Definition: Any process that modulates the frequency, rate or extent of isopentenyl diphosphate biosynthetic process, mevalonate pathway. Subtypes: positive regulation of isopentenyl diphosphate biosynthetic process, mevalonate pathway [GO:1900486], negative regulation of isopentenyl diphosphate biosynthetic process, mevalonate pathway [GO:2001211] Also known as: regulation of Ac-MVA pathway, regulation of acetate-mevalonate pathway, regulation of isopentenyl diphosphate anabolism, mevalonate pathway, regulation of isopentenyl diphosphate formation, mevalonate pathway, regulation of isopentenyl diphosphate synthesis, mevalonate pathway Relationships: is_a regulation of nucleobase-containing compound metabolic process [GO:0019219]; is a type of GO:0019747; is a type of regulation of amide metabolic process [GO:0034248]; is_a regulation of sulfur metabolic process [GO:0042762]; is a type of regulation of small molecule metabolic process [GO:0062012]; is a type of regulation of phospholipid biosynthetic process [GO:0071071]; regulates isopentenyl diphosphate biosynthetic process, mevalonate pathway [GO:0019287] Sources: GOC:al